cellular response to increased oxygen levels [GO:0036295] (biological process) Sources: GOC:al Note: This term should be used when an increase in oxygen levels is not considered a stress response. For a hyperoxic stress response, consider instead 'cellular response to hyperoxia ; GO:0071455'. Also known as: cellular response to raised oxygen levels Definition: Any process that results in a change in state or activity of a cell (in terms of movement, secretion, enzyme production, gene expression, etc.) as a result of a stimulus reflecting an increase in the level of oxygen. Relationships: is a type of GO:0036296; is a type of cellular response to oxygen levels [GO:0071453] Subtypes: GO:0071455